{
  "gene_symbol": "ANKRD61",
  "term_id": "UNKNOWN:0002",
  "gene_name": "Ankyrin repeat domain-containing protein 61",
  "gene": "UniProtKB:A6NGH8",
  "term_label": "Unknown biological process"
}